mitotic spindle formation (spindle phase one) [GO:0061804] (biological process) Definition: The cell cycle process in which the distance is lengthened between poles of the mitotic spindle during mitotic prophase. Also known as: mitotic spindle elongation during mitotic prophase, mitotic spindle elongation during prophase, mitotic spindle elongation during prophase and prometaphase Regulation: regulated by regulation of mitotic spindle formation (spindle phase one) [GO:0110159]; negatively regulated by negative regulation of mitotic spindle formation (spindle phase one) [GO:0110160]; positively regulated by positive regulation of mitotic spindle formation (spindle phase one) [GO:0110161] References: PMID:21920317 Sources: GOC:dph, GOC:vw Relationships: is a type of mitotic spindle organization [GO:0007052]; is part of mitotic spindle elongation [GO:0000022]; is part of mitotic spindle assembly [GO:0090307]; RO_0002092 mitotic prophase [GO:0000088]